establishment of planar polarity of larval imaginal disc epithelium [GO:0042252] (biological process) Relationships: is a type of establishment of planar polarity [GO:0001736] Definition: Coordinated organization of groups of cells in the plane of a larval imaginal disc epithelium, such that they all orient to similar coordinates. Sources: GOC:jl